{
  "gene_symbol": "OR11H4",
  "gene_name": "Olfactory receptor 11H4",
  "term_label": "Unknown molecular function",
  "gene": "UniProtKB:Q8NGC9",
  "term_id": "UNKNOWN:0001"
}